{
  "gene_name": "Tetratricopeptide repeat protein 21A",
  "gene": "UniProtKB:Q8NDW8",
  "term_label": "protein localization to cilium",
  "gene_symbol": "TTC21A",
  "term_id": "GO:0061512"
}